{
  "gene_name": "Ribosome biogenesis protein WDR12",
  "gene_symbol": "WDR12",
  "term_id": "GO:0000463",
  "gene": "UniProtKB:Q9GZL7",
  "term_label": "maturation of LSU-rRNA from tricistronic rRNA transcript (SSU-rRNA, 5.8S rRNA, LSU-rRNA)"
}